{
  "gene_symbol": "SH3GLB2",
  "term_id": "GO:0030674",
  "term_label": "protein-macromolecule adaptor activity",
  "gene_name": "Endophilin-B2",
  "gene": "UniProtKB:Q9NR46"
}